{
  "term_label": "GDP phosphatase activity",
  "gene_symbol": "ENTPD1",
  "gene_name": "Ectonucleoside triphosphate diphosphohydrolase 1",
  "term_id": "GO:0004382",
  "gene": "UniProtKB:P49961"
}